{
  "gene_name": "Transmembrane protein 209",
  "term_id": "UNKNOWN:0002",
  "gene": "UniProtKB:Q96SK2",
  "term_label": "Unknown biological process",
  "gene_symbol": "TMEM209"
}